branching involved in salivary gland morphogenesis [GO:0060445] (biological process) Regulation: RO_0002211 by regulation of branching involved in salivary gland morphogenesis [GO:0060693] Sources: GOC:dph Subtypes: GO:1990632 Definition: The process in which the branching structure of the salivary gland is generated and organized. Relationships: is a type of morphogenesis of a branching epithelium [GO:0061138]; is part of salivary gland morphogenesis [GO:0007435]